{
  "gene": "UniProtKB:Q16585",
  "gene_symbol": "SGCB",
  "term_id": "GO:0042383",
  "term_label": "sarcolemma",
  "gene_name": "Beta-sarcoglycan"
}